Ddb1-Ckn1 complex [GO:0070912] (cellular component) Definition: A heterodimeric nucleotide-excision repair complex that is involved in transcription-coupled repair. The subunits are known as Ddb1 and Ckn1 in S. pombe; Ddb1 contains a motif called the DDB-box that interacts with adaptor proteins for DDB1/cullin 4 ubiquitin ligases. References: PMID:18794354 Relationships: is a type of nucleotide-excision repair complex [GO:0000109]